{
  "gene": "UniProtKB:Q53EV4",
  "gene_symbol": "LRRC23",
  "gene_name": "Leucine-rich repeat-containing protein 23",
  "term_id": "GO:0062177",
  "term_label": "radial spoke assembly"
}